myeloid dendritic cell differentiation [GO:0043011] (biological process) Sources: CL:0000782, GOC:jl Relationships: is a type of myeloid dendritic cell activation [GO:0001773]; is a type of myeloid leukocyte differentiation [GO:0002573]; is a type of dendritic cell differentiation [GO:0097028] Definition: The process in which a monocyte acquires the specialized features of a dendritic cell, an immunocompetent cell of the lymphoid and hemopoietic systems and skin. Subtypes: myeloid dendritic cell differentiation involved in immune response [GO:0002284], Langerhans cell differentiation [GO:0061520]